viral tropism switching [GO:0098678] (biological process) Definition: A process by which the range of hosts which a virus can bind and infect is changed. Examples include phages that switch between types of fibers via the action of a virally encoded invertase. References: PMID:6232613 Sources: VZ:4498 Relationships: is a type of viral process [GO:0016032]